{
  "term_label": "negative regulation of Notch signaling pathway",
  "gene_symbol": "ARRB1",
  "gene": "UniProtKB:P49407",
  "gene_name": "Beta-arrestin-1",
  "term_id": "GO:0045746"
}